carotene catabolic process [GO:0016121] (biological process) Sources: GOC:go_curators Relationships: is a type of carotene metabolic process [GO:0016119]; is a type of terpene catabolic process [GO:0046247] Definition: The chemical reactions and pathways resulting in the breakdown of carotenes, hydrocarbon carotenoids. Also known as: carotene breakdown, carotene catabolism, carotene degradation Subtypes: phytoene catabolic process [GO:1901173], GO:1901176, beta-carotene catabolic process [GO:1901811], beta-zeacarotene catabolic process [GO:1901817], alpha-zeacarotene catabolic process [GO:1901820], delta-carotene catabolic process [GO:1901823]